symbiont-mediated suppression of host JAK-STAT cascade via inhibition of host TYK2 activity [GO:0039574] (biological process) Relationships: is a type of symbiont-mediated suppression of host JAK-STAT cascade [GO:0039514]; is a type of symbiont-mediated suppression of host innate immune response [GO:0052170] References: PMID:16987978, PMID:19085955 Definition: A process in which a symbiont interferes with, inhibits or disrupt a JAK-STAT signal cascade in the host organism by reducing the activity of host TYK2 (tyrosine kinase 2). TYK2 is an intracellular signal-transducing tyrosine kinase involved in numerous cytokines and interferons signaling pathways and transmits the cytokine signal by phosphorylating receptor subunits. Note: This term is for annotation of symbiont proteins that counteract the host innate immune response. Also known as: disruption by virus of host JAK-STAT cascade via inhibition of host TYK2 activity, suppression by virus of host JAK-STAT cascade via inhibition of host TYK2 activity, suppression by virus of host TYK2 activity, suppression by virus of host non-receptor tyrosine-protein kinase TYK2 activity